lymphocyte differentiation [GO:0030098] (biological process) Note: Note that immunologists typically use the word 'development' to refer to cells of B or T cell lineages undergoing the process that GO describes as 'cell differentiation'. Subtypes: natural killer cell differentiation [GO:0001779], B cell differentiation [GO:0030183], T cell differentiation [GO:0030217] Definition: The process in which a relatively unspecialized precursor cell acquires specialized features of a lymphocyte. A lymphocyte is a leukocyte commonly found in the blood and lymph that has the characteristics of a large nucleus, a neutral staining cytoplasm, and prominent heterochromatin. Regulation: regulated by regulation of lymphocyte differentiation [GO:0045619]; RO_0002212 by negative regulation of lymphocyte differentiation [GO:0045620]; positively regulated by positive regulation of lymphocyte differentiation [GO:0045621] Sources: CL:0000542, GOC:go_curators Also known as: lymphocyte cell differentiation, lymphocytic blood cell differentiation, lymphocyte development Relationships: is a type of lymphocyte activation [GO:0046649]; is a type of GO:1903131